{
  "gene_symbol": "TLR6",
  "term_label": "Toll-like receptor 2 binding",
  "term_id": "GO:0035663",
  "gene_name": "Toll-like receptor 6",
  "gene": "UniProtKB:Q9Y2C9"
}